{
  "gene_symbol": "SLCO2B1",
  "gene_name": "Solute carrier organic anion transporter family member 2B1",
  "gene": "UniProtKB:O94956",
  "term_label": "bile acid transmembrane transporter activity",
  "term_id": "GO:0015125"
}